{
  "gene_symbol": "JHY",
  "term_label": "brain development",
  "gene": "UniProtKB:Q6NUN7",
  "term_id": "GO:0007420",
  "gene_name": "Jhy protein homolog"
}